{
  "gene_symbol": "TRIM29",
  "gene_name": "Tripartite motif-containing protein 29",
  "gene": "UniProtKB:Q14134",
  "term_label": "Unknown cellular component",
  "term_id": "UNKNOWN:0003"
}